{
  "gene_symbol": "ASZ1",
  "gene": "UniProtKB:Q8WWH4",
  "gene_name": "Ankyrin repeat, SAM and basic leucine zipper domain-containing protein 1",
  "term_id": "GO:0071546",
  "term_label": "pi-body"
}